{
  "term_id": "GO:0016477",
  "term_label": "cell migration",
  "gene": "UniProtKB:Q6ZW31",
  "gene_symbol": "SYDE1",
  "gene_name": "Rho GTPase-activating protein SYDE1"
}